regulation of action potential firing pattern [GO:0099608] (biological process) Relationships: is a type of GO:0098900; RO_0002211 spike train [GO:0098874] Definition: Any process that regulates the temporal pattern of a sequence of action potentials in a neuron. Sources: ISBN:978-0071390118 Also known as: spike train sculpting